peptidyl-leucine modification [GO:0018204] (biological process) Relationships: is a type of GO:0018193 Sources: GOC:go_curators Definition: The modification of peptidyl-leucine.